{
  "gene_symbol": "CLN6",
  "gene": "UniProtKB:Q9NWW5",
  "term_id": "GO:0007040",
  "gene_name": "Ceroid-lipofuscinosis neuronal protein 6",
  "term_label": "lysosome organization"
}